{
  "term_id": "GO:0009897",
  "gene_name": "GDNF family receptor alpha-1",
  "gene_symbol": "GFRA1",
  "term_label": "external side of plasma membrane",
  "gene": "UniProtKB:P56159"
}